{
  "gene_name": "Kinesin-like protein KIF11",
  "gene_symbol": "KIF11",
  "term_id": "GO:0005634",
  "term_label": "nucleus",
  "gene": "UniProtKB:P52732"
}